ribonucleoside bisphosphate metabolic process [GO:0033875] (BP) Relationships: is a type of GO:0033865 Sources: GOC:mah, GOC:pde Subtypes: GO:0034030, GO:0034031, purine ribonucleoside bisphosphate metabolic process [GO:0034035] Also known as: ribonucleoside bisphosphate metabolism Definition: The chemical reactions and pathways involving a ribonucleoside bisphosphate, a compound consisting of a nucleobase linked to a ribose sugar esterified with one phosphate group attached to each of two different hydroxyl groups on the sugar.